{
  "gene_name": "Sodium_potassium-transporting ATPase subunit alpha-1",
  "gene": "UniProtKB:P05023",
  "gene_symbol": "ATP1A1",
  "term_label": "P-type sodium:potassium-exchanging transporter activity",
  "term_id": "GO:0005391"
}